behavioral response to cocaine [GO:0048148] (BP) Relationships: is a type of adult behavior [GO:0030534]; is part of response to cocaine [GO:0042220] Sources: GOC:jid Definition: Any process that results in a change in the behavior of an organism as a result of a cocaine stimulus. Also known as: behavioural response to cocaine